{
  "gene_symbol": "GNB1",
  "term_label": "G protein-coupled receptor signaling pathway",
  "gene_name": "Guanine nucleotide-binding protein G(I)_G(S)_G(T) subunit beta-1",
  "term_id": "GO:0007186",
  "gene": "UniProtKB:P62873"
}